{
  "term_id": "GO:0007031",
  "term_label": "peroxisome organization",
  "gene_symbol": "ABCD3",
  "gene": "UniProtKB:P28288",
  "gene_name": "ATP-binding cassette sub-family D member 3"
}